{
  "gene_symbol": "MT1X",
  "gene_name": "Metallothionein-1X",
  "gene": "UniProtKB:P80297",
  "term_id": "GO:0010273",
  "term_label": "detoxification of copper ion"
}